positive regulation of cellular response to very-low-density lipoprotein particle stimulus [GO:1905889] (biological process) References: PMID:7592957 Sources: GOC:TermGenie, GOC:aruk, GOC:bc, GO_REF:0000058 Definition: Any process that activates or increases the frequency, rate or extent of cellular response to very-low-density lipoprotein particle stimulus. Relationships: is a type of GO:0048522; is a type of positive regulation of response to stimulus [GO:0048584]; is a type of regulation of cellular response to very-low-density lipoprotein particle stimulus [GO:1905890]; positively regulates cellular response to very-low-density lipoprotein particle stimulus [GO:0090731] Also known as: positive regulation of cellular response to VLDL particle stimulus, up regulation of cellular response to VLDL particle stimulus, up regulation of cellular response to very-low-density lipoprotein particle stimulus, up-regulation of cellular response to VLDL particle stimulus, up-regulation of cellular response to very-low-density lipoprotein particle stimulus, upregulation of cellular response to VLDL particle stimulus, upregulation of cellular response to very-low-density lipoprotein particle stimulus, activation of cellular response to VLDL particle stimulus, activation of cellular response to very-low-density lipoprotein particle stimulus